{
  "term_label": "dorsal/ventral pattern formation",
  "gene_symbol": "BMPR1A",
  "gene": "UniProtKB:P36894",
  "term_id": "GO:0009953",
  "gene_name": "Bone morphogenetic protein receptor type-1A"
}